nematosome [GO:0097417] (cellular component) Relationships: is a type of inclusion body [GO:0016234] Definition: Cytoplasmic, ball-like inclusion resembling a nucleolus and consisting of a convoluted network of electron-opaque strands embedded in a less dense matrix. It measures approximately 0.9 microns and lacks a limiting membrane. Its strands (diameter = 400-600 A) appear to be made of an entanglement of tightly packed filaments and particles approximately 25-50 A thick. Cytochemical studies suggest the presence of nonhistone proteins and some RNA. Usually only one such structure is present in a cell, and it appears to occur in most ganglion cells. Although they can be seen anywhere in the cell body, nematosomes are typically located in the perinuclear cytoplasm, where they are often associated with smooth-surfaced and coated vesicles. References: PMID:5458990 Sources: NIF_Subcellular:sao138430598